{
  "gene_name": "Nitric oxide synthase, inducible",
  "term_id": "GO:0006527",
  "term_label": "L-arginine catabolic process",
  "gene_symbol": "NOS2",
  "gene": "UniProtKB:P35228"
}